galactarate dehydratase activity [GO:0008867] (molecular function) Definition: Catalysis of the reaction: galactarate = 5-dehydro-4-deoxy-D-glucarate + H2O. Also known as: D-galactarate hydro-lyase (5-dehydro-4-deoxy-D-glucarate-forming), D-galactarate hydro-lyase activity Sources: EC:4.2.1.42, RHEA:16005 Relationships: is a type of hydro-lyase activity [GO:0016836]